{
  "gene": "UniProtKB:O15066",
  "term_id": "GO:0005874",
  "term_label": "microtubule",
  "gene_symbol": "KIF3B",
  "gene_name": "Kinesin-like protein KIF3B"
}